olfactory placode formation [GO:0030910] (biological process) Relationships: is a type of ectodermal placode formation [GO:0060788]; BFO_0000050 nose development [GO:0043584]; BFO_0000050 GO:0071699 Definition: The formation of a thickening of the neural ectoderm in the head region of the vertebrate embryo which develops into the olfactory region of the nasal cavity. Sources: GOC:dgh